{
  "gene_name": "Catenin alpha-3",
  "gene_symbol": "CTNNA3",
  "gene": "UniProtKB:Q9UI47",
  "term_id": "GO:0098609",
  "term_label": "cell-cell adhesion"
}